Lewy body-like hyaline inclusion [GO:0097416] (cellular component) Also known as: LBHI Definition: Cytoplasmic inclusion found in neurons. It consists of filaments and granular materials, exhibits a dense core with a rough peripheral halo and lacks a limiting membrane. The filaments of these inclusions are composed of approximately 15-25 nm granule-coated fibrils in association with normal 10-nm neurofilaments. References: PMID:18026741 Sources: NIF_Subcellular:nlx_subcell_20090105 Relationships: is a type of inclusion body [GO:0016234]